{
  "term_label": "synaptonemal complex assembly",
  "gene_name": "Testis-expressed protein 12",
  "gene_symbol": "TEX12",
  "gene": "UniProtKB:Q9BXU0",
  "term_id": "GO:0007130"
}